{
  "term_label": "actin filament organization",
  "term_id": "GO:0007015",
  "gene_symbol": "CORO1C",
  "gene": "UniProtKB:Q9ULV4",
  "gene_name": "Coronin-1C"
}